{
  "gene_symbol": "NEK11",
  "gene": "UniProtKB:Q8NG66",
  "term_label": "regulation of mitotic cell cycle phase transition",
  "term_id": "GO:1901990",
  "gene_name": "Serine_threonine-protein kinase Nek11"
}